{
  "term_id": "GO:0032869",
  "term_label": "cellular response to insulin stimulus",
  "gene_symbol": "PKLR",
  "gene_name": "Pyruvate kinase PKLR",
  "gene": "UniProtKB:P30613"
}